{
  "term_label": "Unknown molecular function",
  "gene_name": "Probable ATP-dependent RNA helicase DDX27",
  "term_id": "UNKNOWN:0001",
  "gene_symbol": "DDX27",
  "gene": "UniProtKB:Q96GQ7"
}